positive regulation of gamma-delta T cell proliferation [GO:0046648] (BP) Sources: GOC:ai Also known as: positive regulation of gamma-delta T lymphocyte proliferation, positive regulation of gamma-delta T-cell proliferation, positive regulation of gamma-delta T-lymphocyte proliferation, up regulation of gamma-delta T cell proliferation, up-regulation of gamma-delta T cell proliferation, upregulation of gamma-delta T cell proliferation, activation of gamma-delta T cell proliferation, stimulation of gamma-delta T cell proliferation Definition: Any process that activates or increases the frequency, rate or extent of gamma-delta T cell proliferation. Relationships: is a type of GO:0042102; is a type of GO:0046645; is a type of regulation of gamma-delta T cell proliferation [GO:0046646]; positively regulates GO:0046630